oxaloacetate decarboxylase activity [GO:0008948] (molecular function) Also known as: oxalacetic acid decarboxylase activity, oxaloacetate carboxy-lyase (pyruvate-forming), oxalate beta-decarboxylase activity, oxaloacetate beta-decarboxylase activity, oxaloacetate carboxy-lyase activity Definition: Catalysis of the reaction: H+ + oxaloacetate = CO2 + pyruvate. Relationships: is a type of carboxy-lyase activity [GO:0016831] Sources: RHEA:15641